chondroitin sulfate proteoglycan catabolic process [GO:0030207] (biological process) References: PMID:17239763 Relationships: is a type of GO:0030167; is a type of chondroitin sulfate proteoglycan metabolic process [GO:0050654] Definition: The chemical reactions and pathways resulting in the breakdown of chondroitin sulfate proteoglycans, which consist of a core protein linked to a chondroitin sulfate glycosaminoglycan. The chondroitin sulfate chain is composed of the repeating disaccharide unit beta-(1,4)-D-glucuronic acid-beta-(1,3)-N-acetyl-D-galactosamine, the latter of which can be O-sulfated. Also known as: chondroitin sulfate breakdown, chondroitin sulfate catabolism, chondroitin sulfate degradation, chondroitin sulphate catabolic process, chondroitin sulphate catabolism